regulation of sensory perception of pain [GO:0051930] (biological process) Definition: Any process that modulates the frequency, rate or extent of the sensory perception of pain, the series of events required for an organism to receive a painful stimulus, convert it to a molecular signal, and recognize and characterize the signal. Subtypes: negative regulation of sensory perception of pain [GO:1904057], GO:1904058 Sources: GOC:ai Relationships: is a type of regulation of sensory perception [GO:0051931]; regulates sensory perception of pain [GO:0019233]